{
  "term_id": "GO:0009922",
  "term_label": "fatty acid elongase activity",
  "gene": "UniProtKB:A1L3X0",
  "gene_symbol": "ELOVL7",
  "gene_name": "Elongation of very long chain fatty acids protein 7"
}